{
  "term_id": "GO:0005667",
  "gene": "UniProtKB:Q15561",
  "gene_symbol": "TEAD4",
  "gene_name": "Transcriptional enhancer factor TEF-3",
  "term_label": "transcription regulator complex"
}